cytoplasmic side of early endosome membrane [GO:0098559] (cellular component) Also known as: external leaflet of early endosome membrane, external side of early endosome membrane Definition: The side (leaflet) of the early endosome membrane that faces the cytoplasm. Relationships: is a type of cytoplasmic side of endosome membrane [GO:0010009]; is part of early endosome membrane [GO:0031901] Sources: GOC:lr Note: In GO, 'external side' still refers to part of the membrane and does not refer to components beyond (outside of) the membrane.